{
  "term_id": "UNKNOWN:0003",
  "gene_symbol": "FRG2B",
  "gene_name": "Protein FRG2-like-1",
  "gene": "UniProtKB:Q96QU4",
  "term_label": "Unknown cellular component"
}